poly(A) RNA polymerase activity [GO:1990817] (molecular function) Regulation: negatively regulated by GO:1904246; positively regulated by positive regulation of polynucleotide adenylyltransferase activity [GO:1904247]; positively regulated by polynucleotide adenylyltransferase activator activity [GO:1990749] Relationships: is a type of adenylyltransferase activity [GO:0070566] References: PMID:13965521 Sources: RHEA:11332 Also known as: NTP polymerase activity, RNA adenylating enzyme, RNA adenyltransferase activity, RNA adenylyltransferase activity, polynucleotide adenylyltransferase activity, poly(A) polymerase activity Definition: Catalysis of the reaction: ATP + RNA(n) = diphosphate + RNA(n)-3'-adenine ribonucleotide. The primer may be an RNA or DNA fragment, or oligo(A) bearing a 3'-OH terminal group.